{
  "term_id": "GO:0072659",
  "gene": "UniProtKB:A8MUH7",
  "gene_name": "Putative PDZ domain-containing protein PDZK1P1",
  "gene_symbol": "PDZK1P1",
  "term_label": "protein localization to plasma membrane"
}